Mad-Max-mSin3B complex [GO:0070440] (cellular component) Definition: A transcriptional repressor complex that contains a heterodimer of the bHLH-ZIP proteins Mad and Max, plus mSin3B, a homolog of the yeast Sin3p. Relationships: is_a RNA polymerase II transcription repressor complex [GO:0090571] References: PMID:7889570